{
  "term_id": "GO:0000981",
  "gene_name": "GS homeobox 1",
  "gene": "UniProtKB:Q9H4S2",
  "term_label": "DNA-binding transcription factor activity, RNA polymerase II-specific",
  "gene_symbol": "GSX1"
}